{
  "term_id": "GO:0005634",
  "gene": "UniProtKB:P11388",
  "gene_name": "DNA topoisomerase 2-alpha",
  "gene_symbol": "TOP2A",
  "term_label": "nucleus"
}